{
  "gene": "UniProtKB:Q16206",
  "gene_name": "Ecto-NOX disulfide-thiol exchanger 2",
  "gene_symbol": "ENOX2",
  "term_id": "UNKNOWN:0001",
  "term_label": "Unknown molecular function"
}